{
  "gene_symbol": "OCM2",
  "gene": "UniProtKB:P0CE71",
  "term_label": "Unknown biological process",
  "gene_name": "Putative oncomodulin-2",
  "term_id": "UNKNOWN:0002"
}